{
  "gene": "UniProtKB:Q9UQF2",
  "gene_name": "C-Jun-amino-terminal kinase-interacting protein 1",
  "term_label": "JNK cascade",
  "term_id": "GO:0007254",
  "gene_symbol": "MAPK8IP1"
}